DNA hairpin binding [GO:0032448] (molecular function) Sources: GOC:mah, ISBN:0198506732 Relationships: is a type of DNA secondary structure binding [GO:0000217] Definition: Binding to a DNA region containing a hairpin. A hairpin structure forms when a DNA strand folds back on itself and intrachain base pairing occurs between inverted repeat sequences.